{
  "gene": "UniProtKB:Q96LA8",
  "gene_symbol": "PRMT6",
  "gene_name": "Protein arginine N-methyltransferase 6",
  "term_id": "UNKNOWN:0003",
  "term_label": "Unknown cellular component"
}